oxidoreductase activity, acting on the CH-NH2 group of donors, NAD or NADP as acceptor [GO:0016639] (molecular function) Subtypes: glutamate dehydrogenase [NAD(P)+] activity [GO:0004353], valine dehydrogenase (NAD+) activity [GO:0043837], L-erythro-3,5-diaminohexanoate dehydrogenase activity [GO:0047124], GO:0047530, diaminopimelate dehydrogenase activity [GO:0047850], glycine dehydrogenase activity [GO:0047960], GO:0050018, L-leucine dehydrogenase activity [GO:0050049], lysine dehydrogenase activity [GO:0050069], GO:0050132, phenylalanine dehydrogenase activity [GO:0050175], serine 2-dehydrogenase activity [GO:0050282], lysine 6-dehydrogenase activity [GO:0050303], tryptophan dehydrogenase activity [GO:0050363], valine dehydrogenase (NADP+) activity [GO:0050391], dehydroquinate synthase activity [GO:0102042] Sources: GOC:ai Relationships: is a type of oxidoreductase activity, acting on the CH-NH2 group of donors [GO:0016638] Definition: Catalysis of an oxidation-reduction (redox) reaction in which a CH-NH2 group acts as a hydrogen or electron donor and reduces NAD+ or NADP.